{
  "gene_name": "L-lactate dehydrogenase A-like 6A",
  "gene_symbol": "LDHAL6A",
  "term_id": "GO:0004459",
  "term_label": "L-lactate dehydrogenase (NAD+) activity",
  "gene": "UniProtKB:Q6ZMR3"
}